{
  "gene_symbol": "PPP4R4",
  "gene": "UniProtKB:Q6NUP7",
  "term_label": "protein phosphatase regulator activity",
  "term_id": "GO:0019888",
  "gene_name": "Serine_threonine-protein phosphatase 4 regulatory subunit 4"
}